{
  "gene_symbol": "ZNF346",
  "term_id": "UNKNOWN:0003",
  "term_label": "Unknown cellular component",
  "gene_name": "Zinc finger protein 346",
  "gene": "UniProtKB:Q9UL40"
}